maltotetraose transport [GO:2001099] (biological process) Relationships: is a type of tetrasaccharide transport [GO:2001098] Definition: The directed movement of a maltotetraoseacetate into, out of or within a cell, or between cells, by means of some agent such as a transporter or pore. Regulation: regulated by regulation of maltotetraose transport [GO:1900321]; negatively regulated by negative regulation of maltotetraose transport [GO:1900322]; positively regulated by positive regulation of maltotetraose transport [GO:1900323] Sources: GOC:mengo_curators